{
  "gene_symbol": "HMGN2",
  "term_id": "GO:0006325",
  "gene": "UniProtKB:P05204",
  "gene_name": "Non-histone chromosomal protein HMG-17",
  "term_label": "chromatin organization"
}